{
  "term_id": "GO:0061844",
  "gene": "UniProtKB:Q16778",
  "gene_symbol": "H2BC21",
  "term_label": "antimicrobial humoral immune response mediated by antimicrobial peptide",
  "gene_name": "Histone H2B type 2-E"
}